{
  "gene_symbol": "ZNF573",
  "gene": "UniProtKB:Q86YE8",
  "gene_name": "Zinc finger protein 573",
  "term_id": "GO:0005634",
  "term_label": "nucleus"
}